{
  "gene": "UniProtKB:P26441",
  "gene_name": "Ciliary neurotrophic factor",
  "term_id": "GO:0097386",
  "gene_symbol": "CNTF",
  "term_label": "glial cell projection"
}